regulation of protein localization to adherens junction [GO:1904702] (biological process) Definition: Any process that modulates the frequency, rate or extent of protein localization to adherens junction. An adherens junction is a cell-cell junction composed of the epithelial cadherin-catenin complex at which the cytoplasmic face of the plasma membrane is attached to actin filaments. References: PMID:26412237 Sources: GOC:TermGenie, GOC:aruk, GOC:bc, GOC:kmv, GO_REF:0000058 Relationships: is a type of regulation of protein localization to cell-cell junction [GO:0150106]; regulates GO:0071896 Subtypes: negative regulation of protein localization to adherens junction [GO:1904703], positive regulation of protein localization to adherens junction [GO:1904704] Also known as: regulation of protein localisation in cell-cell adherens junction, regulation of protein localisation to cell-cell adherens junction, regulation of protein localization in cell-cell adherens junction